{
  "term_id": "GO:0007254",
  "term_label": "JNK cascade",
  "gene": "UniProtKB:O43283",
  "gene_name": "Mitogen-activated protein kinase kinase kinase 13",
  "gene_symbol": "MAP3K13"
}